{
  "gene_name": "Uncharacterized protein C4orf3",
  "gene": "UniProtKB:Q8WVX3",
  "term_id": "UNKNOWN:0001",
  "term_label": "Unknown molecular function",
  "gene_symbol": "C4orf3"
}